{
  "gene_name": "Dipeptidyl peptidase 8",
  "gene": "UniProtKB:Q6V1X1",
  "gene_symbol": "DPP8",
  "term_id": "UNKNOWN:0003",
  "term_label": "Unknown cellular component"
}